regulation of macrophage differentiation [GO:0045649] (biological process) Sources: GOC:go_curators Definition: Any process that modulates the frequency, rate or extent of macrophage differentiation. Relationships: is a type of regulation of myeloid leukocyte differentiation [GO:0002761]; regulates macrophage differentiation [GO:0030225] Subtypes: regulation of microglia differentiation [GO:0014006], negative regulation of macrophage differentiation [GO:0045650], positive regulation of macrophage differentiation [GO:0045651]